{
  "term_label": "regulation of transcription by RNA polymerase II",
  "gene": "UniProtKB:Q96NJ6",
  "term_id": "GO:0006357",
  "gene_name": "Zinc finger protein 3 homolog",
  "gene_symbol": "ZFP3"
}